{
  "term_label": "catalytic step 2 spliceosome",
  "term_id": "GO:0071013",
  "gene": "UniProtKB:P38919",
  "gene_name": "Eukaryotic initiation factor 4A-III",
  "gene_symbol": "EIF4A3"
}